{
  "term_id": "GO:0000978",
  "gene_name": "Zinc finger and BTB domain-containing protein 43",
  "gene": "UniProtKB:O43298",
  "gene_symbol": "ZBTB43",
  "term_label": "RNA polymerase II cis-regulatory region sequence-specific DNA binding"
}